RES complex [GO:0070274] (cellular component) Definition: A protein complex that is required for efficient splicing, and prevents leakage of unspliced pre-mRNAs from the nucleus (named for pre-mRNA REtention and Splicing). In Saccharomyces, the complex consists of Ist3p, Bud13p, and Pml1p. References: PMID:15565172, PMID:18809678, PMID:19010333, PMID:19033360 Also known as: pre-mRNA retention and splicing complex Relationships: is_a nuclear protein-containing complex [GO:0140513]